{
  "term_label": "Unknown cellular component",
  "gene_name": "Lysosomal protective protein",
  "gene_symbol": "CTSA",
  "term_id": "UNKNOWN:0003",
  "gene": "UniProtKB:P10619"
}